{
  "term_id": "GO:0042572",
  "gene": "UniProtKB:Q8N3Y7",
  "gene_name": "Epidermal retinol dehydrogenase 2",
  "gene_symbol": "SDR16C5",
  "term_label": "retinol metabolic process"
}